{
  "term_id": "GO:0035014",
  "term_label": "phosphatidylinositol 3-kinase regulator activity",
  "gene_name": "WD repeat-containing protein 81",
  "gene": "UniProtKB:Q562E7",
  "gene_symbol": "WDR81"
}